{
  "gene_name": "StAR-related lipid transfer protein 4",
  "gene_symbol": "STARD4",
  "gene": "UniProtKB:Q96DR4",
  "term_label": "cholesterol import",
  "term_id": "GO:0070508"
}